positive regulation of cytoplasmic translational elongation through polyproline stretches [GO:1903272] (biological process) Definition: Any process that activates or increases the frequency, rate or extent of cytoplasmic translational elongation through polyproline stretches. Also known as: up regulation of cytoplasmic translational elongation through polyproline stretches, up-regulation of cytoplasmic translational elongation through polyproline stretches, upregulation of cytoplasmic translational elongation through polyproline stretches, activation of cytoplasmic translational elongation through polyproline stretches References: PMID:24923804 Sources: GOC:TermGenie, GO_REF:0000058 Relationships: is a type of positive regulation of cytoplasmic translational elongation [GO:1900249]; is a type of regulation of cytoplasmic translational elongation through polyproline stretches [GO:1903270]; positively regulates cytoplasmic translational elongation through polyproline stretches [GO:0097622]